carnitine O-acyltransferase activity [GO:0016406] (molecular function) Relationships: is a type of GO:0008374 Sources: GOC:ai Subtypes: GO:0004092, carnitine O-palmitoyltransferase activity [GO:0004095], carnitine O-octanoyltransferase activity [GO:0008458] Definition: Catalysis of the transfer of an acyl group to an oxygen atom on the carnitine molecule.